{
  "term_id": "UNKNOWN:0001",
  "term_label": "Unknown molecular function",
  "gene_name": "COP9 signalosome complex subunit 3",
  "gene_symbol": "COPS3",
  "gene": "UniProtKB:Q9UNS2"
}